CHD-type complex [GO:0090545] (CC) References: PMID:17350655 Sources: GOC:krc, GOC:tb Relationships: is a type of SWI/SNF superfamily-type complex [GO:0070603] Subtypes: GO:0016581 Definition: A SWI/SNF-type complex that contains a subunit from the CHD(Chromodomain helicase DNA-binding) family. The CHD family is characterized by two signature sequence motifs: tandem chromodomains located in the N-terminal region, and the SNF2-like ATPase domain located in the central region of the protein structure.